{
  "gene_name": "Ankyrin repeat and SOCS box protein 2",
  "term_id": "GO:0005737",
  "gene": "UniProtKB:Q96Q27",
  "term_label": "cytoplasm",
  "gene_symbol": "ASB2"
}